{
  "gene_symbol": "MRPS14",
  "term_label": "structural constituent of ribosome",
  "gene_name": "Small ribosomal subunit protein uS14m",
  "term_id": "GO:0003735",
  "gene": "UniProtKB:O60783"
}